{
  "gene_symbol": "NPHP3",
  "term_id": "GO:0060026",
  "gene": "UniProtKB:Q7Z494",
  "term_label": "convergent extension",
  "gene_name": "Nephrocystin-3"
}